interleukin-13 receptor activity [GO:0016515] (molecular function) Sources: GOC:jl, GOC:signaling Also known as: IL-13 receptor activity, IL-13R Relationships: is a type of cytokine receptor activity [GO:0004896]; is part of interleukin-13-mediated signaling pathway [GO:0035772]; has part interleukin-13 binding [GO:0019973] Definition: Combining with interleukin-13 and transmitting the signal from one side of the membrane to the other to initiate a change in cell activity.